{
  "gene_name": "G patch domain-containing protein 2-like",
  "gene": "UniProtKB:Q9NWQ4",
  "term_label": "nucleus",
  "gene_symbol": "GPATCH2L",
  "term_id": "GO:0005634"
}